{
  "gene": "UniProtKB:Q92636",
  "term_label": "Unknown cellular component",
  "term_id": "UNKNOWN:0003",
  "gene_name": "Protein FAN",
  "gene_symbol": "NSMAF"
}